{
  "gene_name": "Serine_threonine-protein phosphatase 2A 56 kDa regulatory subunit epsilon isoform",
  "term_label": "nucleus",
  "gene": "UniProtKB:Q16537",
  "term_id": "GO:0005634",
  "gene_symbol": "PPP2R5E"
}